{
  "gene_name": "Cerebral cavernous malformations 2 protein",
  "gene": "UniProtKB:Q9BSQ5",
  "gene_symbol": "CCM2",
  "term_label": "Unknown molecular function",
  "term_id": "UNKNOWN:0001"
}